{
  "term_id": "GO:0050821",
  "gene_symbol": "BAG3",
  "term_label": "protein stabilization",
  "gene": "UniProtKB:O95817",
  "gene_name": "BAG family molecular chaperone regulator 3"
}